{
  "term_label": "transcription coregulator activity",
  "term_id": "GO:0003712",
  "gene_name": "Histone deacetylase complex subunit SAP30",
  "gene": "UniProtKB:O75446",
  "gene_symbol": "SAP30"
}